{
  "gene_symbol": "CADM4",
  "term_label": "homophilic cell-cell adhesion",
  "term_id": "GO:0007156",
  "gene_name": "Cell adhesion molecule 4",
  "gene": "UniProtKB:Q8NFZ8"
}